{
  "gene_symbol": "NDST3",
  "gene_name": "Bifunctional heparan sulfate N-deacetylase_N-sulfotransferase 3",
  "gene": "UniProtKB:O95803",
  "term_label": "heparan sulfate proteoglycan biosynthetic process",
  "term_id": "GO:0015012"
}